{
  "gene": "UniProtKB:Q9P2E2",
  "term_id": "GO:0005815",
  "gene_symbol": "KIF17",
  "gene_name": "Kinesin-like protein KIF17",
  "term_label": "microtubule organizing center"
}